{
  "gene_symbol": "SLC6A4",
  "gene_name": "Sodium-dependent serotonin transporter",
  "gene": "UniProtKB:P31645",
  "term_id": "GO:0051610",
  "term_label": "serotonin uptake"
}